{
  "gene_symbol": "KRTAP5-6",
  "term_label": "Unknown molecular function",
  "gene_name": "Keratin-associated protein 5-6",
  "gene": "UniProtKB:Q6L8G9",
  "term_id": "UNKNOWN:0001"
}